{
  "gene_symbol": "DPCD",
  "gene_name": "Protein DPCD",
  "gene": "UniProtKB:Q9BVM2",
  "term_id": "UNKNOWN:0003",
  "term_label": "Unknown cellular component"
}